{
  "term_id": "GO:0045165",
  "term_label": "cell fate commitment",
  "gene_symbol": "WNT7A",
  "gene": "UniProtKB:O00755",
  "gene_name": "Protein Wnt-7a"
}